{
  "gene_name": "Protein EVI2B",
  "gene_symbol": "EVI2B",
  "gene": "UniProtKB:P34910",
  "term_label": "positive regulation of neutrophil differentiation",
  "term_id": "GO:0045660"
}